{
  "gene": "UniProtKB:O95848",
  "gene_name": "Uridine diphosphate glucose pyrophosphatase NUDT14",
  "term_id": "GO:0019693",
  "term_label": "ribose phosphate metabolic process",
  "gene_symbol": "NUDT14"
}